gamma-aminobutyric acid:proton symporter activity [GO:0015495] (molecular function) Also known as: 4-aminobutanoate:hydrogen symporter activity, 4-aminobutanoate:proton symporter activity, 4-aminobutyrate:hydrogen symporter activity, 4-aminobutyrate:proton symporter activity, GABA:hydrogen symporter activity, GABA:proton symporter activity, gamma-aminobutyric acid permease activity, gamma-aminobutyric acid:hydrogen symporter activity Sources: TC:2.A.18.5.1, TC:2.A.3.1.4, TC:2.A.3.4.2 Note: See also the molecular function term 'neurotransmitter transporter activity ; GO:0005326'. Definition: Enables the transfer of a solute or solutes from one side of a membrane to the other according to the reaction: gamma-aminobutyric acid(out) + H+(out) = gamma-aminobutyric acid(in) + H+(in). Relationships: is_a amino acid:proton symporter activity [GO:0005280]; is a type of gamma-aminobutyric acid transmembrane transporter activity [GO:0015185]; is a type of secondary active monocarboxylate transmembrane transporter activity [GO:0015355]